{
  "gene_name": "Granulocyte-macrophage colony-stimulating factor receptor subunit alpha",
  "gene": "UniProtKB:P15509",
  "term_id": "GO:0046427",
  "term_label": "positive regulation of receptor signaling pathway via JAK-STAT",
  "gene_symbol": "CSF2RA"
}